positive regulation of neuromuscular synaptic transmission [GO:1900075] (biological process) Sources: GOC:TermGenie, GOC:kmv Also known as: activation of neuromuscular synaptic transmission, up regulation of neuromuscular synaptic transmission, up-regulation of neuromuscular synaptic transmission, upregulation of neuromuscular synaptic transmission Relationships: is a type of GO:0050806; is a type of GO:1900073; positively regulates GO:0007274 Definition: Any process that activates or increases the frequency, rate or extent of neuromuscular synaptic transmission.